regulation of hexadecanal biosynthetic process [GO:1900902] (biological process) Definition: Any process that modulates the frequency, rate or extent of hexadecanal biosynthetic process. Subtypes: GO:1900903, positive regulation of hexadecanal biosynthetic process [GO:1900904] Sources: GOC:TermGenie, GOC:mengo_curators Relationships: is a type of GO:0009889; regulates hexadecanal biosynthetic process [GO:0006634] Also known as: regulation of hexadecanal anabolism, regulation of hexadecanal biosynthesis, regulation of hexadecanal formation, regulation of hexadecanal synthesis, regulation of palmitaldehyde biosynthesis, regulation of palmitaldehyde biosynthetic process